{
  "term_id": "GO:0097125",
  "gene_name": "G2_mitotic-specific cyclin-B1",
  "gene": "UniProtKB:P14635",
  "term_label": "cyclin B1-CDK1 complex",
  "gene_symbol": "CCNB1"
}